{
  "gene_name": "Olfactory receptor 5AR1",
  "gene": "UniProtKB:Q8NGP9",
  "term_id": "UNKNOWN:0003",
  "term_label": "Unknown cellular component",
  "gene_symbol": "OR5AR1"
}